{
  "gene_name": "Integrin beta-5",
  "gene": "UniProtKB:P18084",
  "term_id": "GO:0009986",
  "gene_symbol": "ITGB5",
  "term_label": "cell surface"
}